{
  "gene_symbol": "SCUBE1",
  "gene_name": "Signal peptide, CUB and EGF-like domain-containing protein 1",
  "term_id": "UNKNOWN:0001",
  "term_label": "Unknown molecular function",
  "gene": "UniProtKB:Q8IWY4"
}